{
  "gene_symbol": "CHRND",
  "term_label": "skeletal muscle contraction",
  "gene": "UniProtKB:Q07001",
  "term_id": "GO:0003009",
  "gene_name": "Acetylcholine receptor subunit delta"
}